{
  "gene_name": "Solute carrier family 12 member 5",
  "gene": "UniProtKB:Q9H2X9",
  "gene_symbol": "SLC12A5",
  "term_id": "GO:0006884",
  "term_label": "cell volume homeostasis"
}